tetrahydrofolate metabolic process [GO:0046653] (biological process) Subtypes: 10-formyltetrahydrofolate metabolic process [GO:0009256], tetrahydrofolate interconversion [GO:0035999], tetrahydrofolate biosynthetic process [GO:0046654] Also known as: tetrahydrofolate metabolism Relationships: is a type of folic acid-containing compound metabolic process [GO:0006760] Definition: The chemical reactions and pathways involving tetrahydrofolate, 5,6,7,8-tetrahydrofolic acid, a folate derivative bearing additional hydrogens on the pterin group. Sources: ISBN:0198506732